{
  "gene": "UniProtKB:Q15796",
  "term_label": "anatomical structure morphogenesis",
  "term_id": "GO:0009653",
  "gene_name": "Mothers against decapentaplegic homolog 2",
  "gene_symbol": "SMAD2"
}